acetoin catabolic process [GO:0045150] (biological process) Also known as: acetoin breakdown, acetoin catabolism, acetoin degradation Sources: GOC:mlg Definition: The chemical reactions and pathways resulting in the breakdown of acetoin, 3-hydroxy-2-butanone. Relationships: is a type of ketone catabolic process [GO:0042182]; is a type of acetoin metabolic process [GO:0045149]; is a type of alcohol catabolic process [GO:0046164]